malate:sodium symporter activity [GO:0043882] (molecular function) Relationships: is a type of malate transmembrane transporter activity [GO:0015140]; is a type of sodium:dicarboxylate symporter activity [GO:0017153] References: PMID:10903309 Sources: GOC:jl Also known as: malate/sodium cotransporter activity, malate:sodium cotransporter activity, sodium-dependent malate transporter, Na(+)-malate symporter activity, Na+:malate symporter activity, malate Na(+) symporter activity, malate-sodium symporter activity, malate/sodium symporter activity, malate:Na+ symporter activity, sodium/malate symporter activity, sodium:malate symporter activity Definition: Enables the transfer of a solute or solutes from one side of a membrane to the other according to the reaction: malate(out) + Na+(out) = malate(in) + Na+(in).